follicle-stimulating hormone complex [GO:0016914] (cellular component) Definition: A gonadotrophic glycoprotein hormone secreted, in mammals, by the anterior pituitary gland; consists of alpha and beta subunits, the latter of which confers hormonal specificity. Sources: ISBN:0198547684 Also known as: FSH complex, follicle stimulating hormone complex Relationships: is a type of pituitary gonadotropin complex [GO:0061696]